positive regulation of cell communication by chemical coupling [GO:0010652] (biological process) Sources: GOC:dph, GOC:kmv, GOC:tb Definition: Any process that increases the frequency, rate or extent of cell communication via chemical coupling. Cell communication by chemical coupling is the process that mediates signaling interactions between one cell and another cell by the transfer of small, water-soluble molecules or metabolites between their adjacent cytoplasms via intercellular protein channels. Relationships: is a type of regulation of cell communication by chemical coupling [GO:0010645]; is a type of positive regulation of cell communication [GO:0010647]; positively regulates cell communication by chemical coupling [GO:0010643]